positive regulation of Wnt protein secretion [GO:0061357] (BP) Relationships: is a type of positive regulation of cell communication [GO:0010647]; is a type of positive regulation of signaling [GO:0023056]; is a type of positive regulation of protein secretion [GO:0050714]; is a type of regulation of Wnt protein secretion [GO:0061356]; positively regulates Wnt protein secretion [GO:0061355] References: PMID:19223472 Sources: GOC:bf Definition: Any process that activates or increases the frequency, rate or extent of the controlled release of a Wnt protein from a cell.